{
  "gene": "UniProtKB:Q8TB72",
  "term_label": "mRNA 3'-UTR binding",
  "gene_symbol": "PUM2",
  "term_id": "GO:0003730",
  "gene_name": "Pumilio homolog 2"
}